{
  "gene_symbol": "ARHGDIA",
  "gene_name": "Rho GDP-dissociation inhibitor 1",
  "gene": "UniProtKB:P52565",
  "term_id": "GO:0005094",
  "term_label": "Rho GDP-dissociation inhibitor activity"
}